{
  "gene_symbol": "ALKAL2",
  "term_id": "GO:0070374",
  "gene_name": "ALK and LTK ligand 2",
  "gene": "UniProtKB:Q6UX46",
  "term_label": "positive regulation of ERK1 and ERK2 cascade"
}